{
  "gene_symbol": "TBL1X",
  "term_label": "regulation of transcription by RNA polymerase II",
  "term_id": "GO:0006357",
  "gene_name": "F-box-like_WD repeat-containing protein TBL1X",
  "gene": "UniProtKB:O60907"
}